{
  "gene_symbol": "LIMK1",
  "gene": "UniProtKB:P53667",
  "gene_name": "LIM domain kinase 1",
  "term_label": "nucleus",
  "term_id": "GO:0005634"
}